methanol-5-hydroxybenzimidazolylcobamide Co-methyltransferase activity [GO:0047152] (molecular function) Definition: Catalysis of the reaction: 5-hydroxybenzimidazolylcobamide + methanol = H2O + Co-methyl-Co-5-hydroxybenzimidazolylcob(I)amide. Note: This function is the first step in the pathway of methanogenesis from methanol. Relationships: is a type of methyltransferase activity [GO:0008168] Also known as: methyltransferase 1, methanol-corrinoid protein Co-methyltransferase, methanol:corrinoid methyltransferase activity, MT 1, MT1, MtaB, methanol cobalamin methyltransferase activity, methanol:5-hydroxybenzimidazolylcobamide Co-methyltransferase activity, methanol:5-hydroxybenzimidazolylcobamide methyltransferase activity References: PMID:6438059 Sources: RHEA:45204